{
  "gene_symbol": "CCT5",
  "gene": "UniProtKB:P48643",
  "term_id": "GO:0005832",
  "gene_name": "T-complex protein 1 subunit epsilon",
  "term_label": "chaperonin-containing T-complex"
}